{
  "term_label": "phosphatidylinositol-3,5-bisphosphate binding",
  "gene_name": "Huntingtin-interacting protein 1",
  "term_id": "GO:0080025",
  "gene": "UniProtKB:O00291",
  "gene_symbol": "HIP1"
}